{
  "gene_name": "NLR family member X1",
  "gene_symbol": "NLRX1",
  "term_id": "GO:0005739",
  "term_label": "mitochondrion",
  "gene": "UniProtKB:Q86UT6"
}